{
  "gene": "UniProtKB:A0A1W2PR82",
  "gene_symbol": "PERCC1",
  "gene_name": "Protein PERCC1",
  "term_label": "Unknown biological process",
  "term_id": "UNKNOWN:0002"
}